{
  "gene_name": "Centrosomal protein of 192 kDa",
  "gene": "UniProtKB:Q8TEP8",
  "term_id": "GO:0005814",
  "gene_symbol": "CEP192",
  "term_label": "centriole"
}